proton-transporting two-sector ATPase complex, catalytic domain [GO:0033178] (cellular component) Relationships: is a type of membrane protein complex [GO:0098796]; is part of GO:0016469 Subtypes: proton-transporting V-type ATPase, V1 domain [GO:0033180] References: PMID:10838056 Sources: GOC:mah Definition: A protein complex that forms part of a proton-transporting two-sector ATPase complex and catalyzes ATP hydrolysis or synthesis. The catalytic domain (F1, V1, or A1) comprises a hexameric catalytic core and a central stalk, and is peripherally associated with the membrane when the two-sector ATPase is assembled.